inter-Golgi transport vesicle membrane [GO:0012509] (cellular component) Also known as: inter-Golgi transport constitutive secretory pathway transport vesicle membrane Sources: GOC:ai Relationships: is a type of transport vesicle membrane [GO:0030658]; is a type of GO:0030663; is part of GO:0030143 Definition: The lipid bilayer surrounding a vesicle transporting substances within the Golgi.